{
  "term_label": "translation initiation factor activity",
  "gene_name": "Eukaryotic translation initiation factor 3 subunit A",
  "gene_symbol": "EIF3A",
  "gene": "UniProtKB:Q14152",
  "term_id": "GO:0003743"
}